{
  "term_label": "cytosol",
  "term_id": "GO:0005829",
  "gene_symbol": "HSP90AB4P",
  "gene": "UniProtKB:Q58FF6",
  "gene_name": "Putative heat shock protein HSP 90-beta 4"
}